{
  "gene_symbol": "UNC119B",
  "gene_name": "Protein unc-119 homolog B",
  "term_id": "GO:0008289",
  "term_label": "lipid binding",
  "gene": "UniProtKB:A6NIH7"
}